positive regulation of eosinophil degranulation [GO:0043311] (BP) Also known as: positive regulation of eosinophil granule exocytosis, up regulation of eosinophil degranulation, up-regulation of eosinophil degranulation, upregulation of eosinophil degranulation, activation of eosinophil degranulation, stimulation of eosinophil degranulation Relationships: is a type of GO:0002888; is a type of positive regulation of leukocyte degranulation [GO:0043302]; is a type of regulation of eosinophil degranulation [GO:0043309]; is a type of GO:0050778; positively regulates eosinophil degranulation [GO:0043308] Definition: Any process that activates or increases the frequency, rate or extent of eosinophil degranulation. Sources: ISBN:0781735149